hydrogenobyrinic acid a,c-diamide synthase (glutamine-hydrolysing) activity [GO:0043802] (molecular function) Relationships: is a type of carbon-nitrogen ligase activity, with glutamine as amido-N-donor [GO:0016884] Definition: Catalysis of the reaction: 2 L-glutamine + 2 ATP + 2 H2O + hydrogenobyrinate = 2 L-glutamate + 2 ADP + 4 H+ + hydrogenobyrinate a,c-diamide + 2 phosphate. Also known as: hydrogenobyrinic acid a,c diamide synthase (glutamine-hydrolysing) activity, hydrogenobyrinic-acid:L-glutamine amido-ligase (AMP-forming), CobB Sources: EC:6.3.5.9, RHEA:12544